{
  "gene": "UniProtKB:Q9UHV5",
  "gene_symbol": "RAPGEFL1",
  "gene_name": "Rap guanine nucleotide exchange factor-like 1",
  "term_label": "plasma membrane",
  "term_id": "GO:0005886"
}